{
  "term_label": "cytoplasm",
  "gene_name": "BLOC-2 complex member HPS5",
  "gene": "UniProtKB:Q9UPZ3",
  "term_id": "GO:0005737",
  "gene_symbol": "HPS5"
}